response to cycloheximide [GO:0046898] (biological process) Also known as: response to actidione Sources: GOC:ef, ISBN:0198506732 Relationships: is a type of response to alcohol [GO:0097305]; is a type of response to ketone [GO:1901654]; is a type of GO:1901698 Definition: Any process that results in a change in state or activity of a cell or an organism (in terms of movement, secretion, enzyme production, gene expression, etc.) as a result of a cycloheximide stimulus. Cycloheximide (actidione) is an antibiotic produced by some Streptomyces species which interferes with protein synthesis in eukaryotes. Subtypes: cellular response to cycloheximide [GO:0071409]